ligase activity, forming carbon-nitrogen bonds [GO:0016879] (molecular function) Subtypes: beta-alanyl amine synthase activity [GO:0003833], CTP synthase activity [GO:0003883], GO:0003921, adenylosuccinate synthase activity [GO:0004019], GO:0004055, biotin carboxylase activity [GO:0004075], biotin--[biotin carboxyl-carrier protein] ligase activity [GO:0004077], carbamoyl-phosphate synthase (ammonia) activity [GO:0004087], formate-tetrahydrofolate ligase activity [GO:0004329], GO:0004516, GO:0004637, urea carboxylase activity [GO:0004847], acid-ammonia (or amide) ligase activity [GO:0016880], acid-amino acid ligase activity [GO:0016881], cyclo-ligase activity [GO:0016882], carbon-nitrogen ligase activity, with glutamine as amido-N-donor [GO:0016884], GO:0016979, GO:0032267, 5-(carboxyamino)imidazole ribonucleotide synthase activity [GO:0034028], GO:0047483, formate-dihydrofolate ligase activity [GO:0047897], GO:0047943, GO:0050260, N-acetyl-L-aspartate-L-glutamate ligase activity [GO:0072590], citrate-L-glutamate ligase activity [GO:0072591], indole-3-acetyl-glycine synthetase activity [GO:0102047], indole-3-acetyl-isoleucine synthetase activity [GO:0102048], GO:0102049 Also known as: other carbon-nitrogen ligase activity Definition: Catalysis of the joining of two molecules, or two groups within a single molecule, via a carbon-nitrogen bond, with the concomitant hydrolysis of the diphosphate bond in ATP or a similar triphosphate. Sources: EC:6.3.-.- Relationships: is a type of GO:0016874